{
  "term_label": "histone H3K36 methyltransferase activity",
  "gene": "UniProtKB:Q86TU7",
  "term_id": "GO:0046975",
  "gene_name": "Actin-histidine N-methyltransferase",
  "gene_symbol": "SETD3"
}